negative regulation of mesenchymal cell proliferation involved in ureter development [GO:0072200] (BP) Also known as: negative regulation of ureter mesenchymal cell proliferation, negative regulation of ureteral mesenchymal cell proliferation Definition: Any process that decreases the frequency, rate or extent of mesenchymal cell proliferation that contributes to the progression of the ureter gland over time. A mesenchymal cell is a cell that normally gives rise to other cells that are organized as three-dimensional masses, rather than sheets. Relationships: is a type of negative regulation of developmental process [GO:0051093]; is_a GO:0051241; is_a regulation of mesenchymal cell proliferation involved in ureter development [GO:0072199]; is a type of negative regulation of mesenchymal cell proliferation [GO:0072201]; RO_0002212 mesenchymal cell proliferation involved in ureter development [GO:0072198] Sources: GOC:mtg_kidney_jan10